regulation of smooth muscle cell proliferation [GO:0048660] (biological process) Relationships: is a type of regulation of cell population proliferation [GO:0042127]; regulates GO:0048659 Subtypes: positive regulation of smooth muscle cell proliferation [GO:0048661], GO:0048662, regulation of vascular associated smooth muscle cell proliferation [GO:1904705] Definition: Any process that modulates the frequency, rate or extent of smooth muscle cell proliferation. Sources: CL:0000192, GOC:ebc Also known as: regulation of SMC proliferation